regulation of phospholipid translocation [GO:0061091] (biological process) Subtypes: positive regulation of phospholipid translocation [GO:0061092], negative regulation of phospholipid translocation [GO:0061093], regulation of phosphatidylserine exposure on apoptotic cell surface [GO:1905780] Definition: Any process that modulates the frequency, rate or extent of the translocation, or flipping, of phospholipid molecules from one monolayer of a membrane bilayer to the opposite monolayer. Relationships: is a type of regulation of cellular component organization [GO:0051128]; is a type of regulation of membrane lipid distribution [GO:0097035]; is a type of GO:2001138; regulates phospholipid translocation [GO:0045332] References: PMID:19966303 Sources: GOC:dph, GOC:jh, GOC:tb